{
  "term_label": "plasma membrane",
  "gene_name": "Probable G-protein coupled receptor 88",
  "gene_symbol": "GPR88",
  "term_id": "GO:0005886",
  "gene": "UniProtKB:Q9GZN0"
}